{
  "gene_symbol": "SLC2A5",
  "gene_name": "Solute carrier family 2, facilitated glucose transporter member 5",
  "term_label": "D-glucose transmembrane transporter activity",
  "gene": "UniProtKB:P22732",
  "term_id": "GO:0055056"
}